{
  "term_label": "clathrin coat assembly",
  "gene_symbol": "FCHO1",
  "gene": "UniProtKB:O14526",
  "term_id": "GO:0048268",
  "gene_name": "F-BAR domain only protein 1"
}